{
  "term_label": "synaptic vesicle clustering",
  "gene_name": "Synapse differentiation-inducing gene protein 1",
  "term_id": "GO:0097091",
  "gene_symbol": "SYNDIG1",
  "gene": "UniProtKB:Q9H7V2"
}